poly-purine tract binding [GO:0070717] (molecular function) Sources: GOC:mah Subtypes: poly(A) binding [GO:0008143], poly(G) binding [GO:0034046] Relationships: is a type of single-stranded RNA binding [GO:0003727] Definition: Binding to a stretch of purines (adenine or guanine) in an RNA molecule.